oxaloacetate transmembrane transporter activity [GO:0015131] (MF) Definition: Enables the transfer of oxaloacetate, the anion of oxobutanedioic acid, from one side of a membrane to the other. Sources: GOC:ai Relationships: is_a GO:0005310; is a type of GO:0015556; is part of oxaloacetate(2-) transmembrane transport [GO:1902356]